{
  "gene": "UniProtKB:Q9BX73",
  "term_id": "UNKNOWN:0002",
  "gene_name": "TM2 domain-containing protein 2",
  "gene_symbol": "TM2D2",
  "term_label": "Unknown biological process"
}